{
  "gene_name": "RNA-binding protein 12B",
  "term_id": "GO:0005654",
  "term_label": "nucleoplasm",
  "gene": "UniProtKB:Q8IXT5",
  "gene_symbol": "RBM12B"
}